galacturonan binding [GO:0048028] (MF) Definition: Binding to a simple or complex galacturonan. Galacturonan is any glycan composed solely of galacturonic acid residues, a specific type of glycuronan, and a constituent of some pectins. Sources: GOC:jid Also known as: polygalacturonide binding Relationships: is a type of polysaccharide binding [GO:0030247] Subtypes: pectin binding [GO:0044589]